{
  "term_label": "cell differentiation",
  "gene_name": "Hepatocyte nuclear factor 4-alpha",
  "gene": "UniProtKB:P41235",
  "term_id": "GO:0030154",
  "gene_symbol": "HNF4A"
}